{
  "gene": "UniProtKB:Q9NSE4",
  "term_label": "mitochondrial translation",
  "gene_name": "Isoleucine--tRNA ligase, mitochondrial",
  "gene_symbol": "IARS2",
  "term_id": "GO:0032543"
}